urate metabolic process [GO:0046415] (biological process) Definition: The chemical reactions and pathways involving urate, the anion of uric acid, 2,6,8-trioxypurine, the end product of purine metabolism in certain mammals and the main excretory product in uricotelic animals. Sources: ISBN:0198506732 Also known as: urate metabolism Relationships: is a type of small molecule metabolic process [GO:0044281]; is a type of purine-containing compound metabolic process [GO:0072521] Subtypes: urate catabolic process [GO:0019628], urate biosynthetic process [GO:0034418]